positive regulation of lateral mesodermal cell fate determination [GO:0048376] (biological process) Relationships: is a type of positive regulation of mesodermal cell fate determination [GO:0048336]; is a type of GO:0048374; positively regulates lateral mesodermal cell fate determination [GO:0048373] Also known as: positive regulation of lateral plate mesodermal cell fate determination, up regulation of lateral mesodermal cell fate determination, up-regulation of lateral mesodermal cell fate determination, upregulation of lateral mesodermal cell fate determination, activation of lateral mesodermal cell fate determination, stimulation of lateral mesodermal cell fate determination Sources: GOC:jid Definition: Any process that activates or increases the frequency, rate or extent of lateral mesoderm cell fate determination.